{
  "gene_symbol": "PARP1",
  "gene_name": "Poly [ADP-ribose] polymerase 1",
  "gene": "UniProtKB:P09874",
  "term_label": "double-strand break repair",
  "term_id": "GO:0006302"
}